{
  "term_id": "GO:0005634",
  "term_label": "nucleus",
  "gene_name": "Nuclear receptor coactivator 3",
  "gene": "UniProtKB:Q9Y6Q9",
  "gene_symbol": "NCOA3"
}